{
  "term_id": "GO:0000724",
  "term_label": "double-strand break repair via homologous recombination",
  "gene": "UniProtKB:Q96B01",
  "gene_name": "RAD51-associated protein 1",
  "gene_symbol": "RAD51AP1"
}